{
  "gene_name": "Neprilysin",
  "gene": "UniProtKB:P08473",
  "gene_symbol": "MME",
  "term_id": "GO:0097242",
  "term_label": "amyloid-beta clearance"
}